{
  "gene_name": "Histone deacetylase complex subunit SAP30",
  "term_id": "GO:0000118",
  "term_label": "histone deacetylase complex",
  "gene_symbol": "SAP30",
  "gene": "UniProtKB:O75446"
}